{
  "term_id": "GO:0030553",
  "gene_name": "Cyclic nucleotide-gated cation channel alpha-4",
  "gene_symbol": "CNGA4",
  "term_label": "cGMP binding",
  "gene": "UniProtKB:Q8IV77"
}